{
  "term_id": "GO:0009311",
  "gene": "UniProtKB:P17050",
  "term_label": "oligosaccharide metabolic process",
  "gene_name": "Alpha-N-acetylgalactosaminidase",
  "gene_symbol": "NAGA"
}